{
  "term_label": "membrane",
  "term_id": "GO:0016020",
  "gene_symbol": "SEC62",
  "gene_name": "Translocation protein SEC62",
  "gene": "UniProtKB:Q99442"
}